{
  "term_label": "sodium:proton antiporter activity",
  "gene_symbol": "SLC9C1",
  "gene": "UniProtKB:Q4G0N8",
  "term_id": "GO:0015385",
  "gene_name": "Sodium_hydrogen exchanger 10"
}